ATP-dependent protein-DNA complex displacement activity [GO:0061995] (molecular function) Also known as: ATP-dependent protein-nucleic acid complex displacement activity Relationships: is a type of ATP-dependent protein-DNA unloader activity [GO:0140083] References: PMID:18593879 Definition: An activity that displaces proteins or protein complexes from DNA, sometimes in a 'wire stripping' fashion, driven by ATP hydrolysis.